{
  "gene_symbol": "VPS39",
  "term_label": "small GTPase binding",
  "gene_name": "Vam6_Vps39-like protein",
  "gene": "UniProtKB:Q96JC1",
  "term_id": "GO:0031267"
}